{
  "gene_symbol": "RAB11FIP4",
  "term_id": "GO:0032465",
  "gene": "UniProtKB:Q86YS3",
  "gene_name": "Rab11 family-interacting protein 4",
  "term_label": "regulation of cytokinesis"
}